{
  "term_label": "synapse",
  "gene": "UniProtKB:P20309",
  "term_id": "GO:0045202",
  "gene_name": "Muscarinic acetylcholine receptor M3",
  "gene_symbol": "CHRM3"
}